{
  "term_id": "GO:0005737",
  "gene_name": "SUMO-activating enzyme subunit 1",
  "gene_symbol": "SAE1",
  "term_label": "cytoplasm",
  "gene": "UniProtKB:Q9UBE0"
}